{
  "gene_symbol": "PIWIL3",
  "gene": "UniProtKB:Q7Z3Z3",
  "gene_name": "Piwi-like protein 3",
  "term_id": "GO:0004521",
  "term_label": "RNA endonuclease activity"
}